{
  "gene": "UniProtKB:Q7LC44",
  "term_id": "GO:0005198",
  "gene_name": "Activity-regulated cytoskeleton-associated protein",
  "term_label": "structural molecule activity",
  "gene_symbol": "ARC"
}